IP-10 production [GO:0071612] (biological process) Definition: The appearance of IP-10 due to biosynthesis or secretion following a cellular stimulus, resulting in an increase in its intracellular or extracellular levels. Sources: GOC:add, GOC:rv Also known as: CXCL10 production, chemokine (C-C motif) ligand 10 production Relationships: is a type of chemokine production [GO:0032602] Regulation: regulated by regulation of IP-10 production [GO:0071658]; RO_0002212 by negative regulation of IP-10 production [GO:0071659]; positively regulated by GO:0071660